rhamnetin 3-O-methyltransferase activity [GO:0102446] (MF) Sources: RHEA:74763 Definition: Catalysis of the reaction: rhamnetin + S-adenosyl-L-methionine = 3',4',5-trihydroxy-3,7-dimethoxyflavone + H+ + S-adenosyl-L-homocysteine. Relationships: is a type of methyltransferase activity [GO:0008168]